negative regulation of neutrophil degranulation [GO:0043314] (biological process) Definition: Any process that stops, prevents, or reduces the rate of neutrophil degranulation. Also known as: down regulation of neutrophil degranulation, down-regulation of neutrophil degranulation, downregulation of neutrophil degranulation, negative regulation of neutrophil granule exocytosis, inhibition of neutrophil degranulation Relationships: is_a negative regulation of myeloid leukocyte mediated immunity [GO:0002887]; is a type of negative regulation of leukocyte degranulation [GO:0043301]; is a type of regulation of neutrophil degranulation [GO:0043313]; is a type of negative regulation of immune response [GO:0050777]; negatively regulates neutrophil degranulation [GO:0043312] Sources: ISBN:0781735149